tRNA aminoacylation [GO:0043039] (biological process) Relationships: is a type of tRNA metabolic process [GO:0006399]; is a type of amino acid activation [GO:0043038] Also known as: aminoacyl-tRNA biosynthesis, aminoacyl-tRNA biosynthetic process, tRNA charging, amino acid activation Definition: The chemical reactions and pathways by which the various amino acids become bonded to their corresponding tRNAs. The most common route for synthesis of aminoacyl tRNA is by the formation of an ester bond between the 3'-hydroxyl group of the most 3' adenosine of the tRNA and the alpha carboxylic acid group of an amino acid, usually catalyzed by the cognate aminoacyl-tRNA ligase. A given aminoacyl-tRNA ligase aminoacylates all species of an isoaccepting group of tRNA molecules. Subtypes: tRNA aminoacylation for protein translation [GO:0006418], tRNA aminoacylation for nonribosomal peptide biosynthetic process [GO:0043040], asparaginyl-tRNAAsn biosynthesis via transamidation [GO:0070680], glutaminyl-tRNAGln biosynthesis via transamidation [GO:0070681] Sources: GOC:ma, GOC:mah